{
  "gene_name": "Endosome_lysosome-associated apoptosis and autophagy regulator 1",
  "gene_symbol": "ELAPOR1",
  "term_label": "positive regulation of vacuole organization",
  "gene": "UniProtKB:Q6UXG2",
  "term_id": "GO:0044090"
}